response to hormone [GO:0009725] (biological process) Relationships: is a type of response to endogenous stimulus [GO:0009719]; is_a response to chemical [GO:0042221] Subtypes: detection of hormone stimulus [GO:0009720], response to ethylene [GO:0009723], GO:0009733, GO:0009735, response to abscisic acid [GO:0009737], response to gibberellin [GO:0009739], response to brassinosteroid [GO:0009741], response to jasmonic acid [GO:0009753], GO:0032870, response to prostaglandin [GO:0034694], GO:0034698, GO:0043434, response to estrogen [GO:0043627], response to leptin [GO:0044321], response to steroid hormone [GO:0048545], response to parathyroid hormone [GO:0071107], response to thyroid hormone [GO:0097066], GO:1990418, response to growth hormone-releasing hormone [GO:1990864] Definition: Any process that results in a change in state or activity of a cell or an organism (in terms of movement, secretion, enzyme production, gene expression, etc.) as a result of a hormone stimulus. Also known as: response to hormone stimulus, growth regulator Sources: GOC:jl